{
  "term_label": "neuron projection",
  "term_id": "GO:0043005",
  "gene_symbol": "NPY4R2",
  "gene_name": "Neuropeptide Y receptor type 4-2",
  "gene": "UniProtKB:P0DQD5"
}